{
  "term_label": "GTPase activity",
  "term_id": "GO:0003924",
  "gene_symbol": "RAP2C",
  "gene": "UniProtKB:Q9Y3L5",
  "gene_name": "Ras-related protein Rap-2c"
}